{
  "gene": "UniProtKB:Q9Y5F0",
  "gene_name": "Protocadherin beta-13",
  "term_label": "cell adhesion molecule binding",
  "term_id": "GO:0050839",
  "gene_symbol": "PCDHB13"
}